{
  "term_label": "Z disc",
  "gene_name": "PDZ and LIM domain protein 2",
  "gene": "UniProtKB:Q96JY6",
  "gene_symbol": "PDLIM2",
  "term_id": "GO:0030018"
}